{
  "gene_symbol": "SLC3A2",
  "term_id": "UNKNOWN:0001",
  "term_label": "Unknown molecular function",
  "gene_name": "4F2 cell-surface antigen heavy chain",
  "gene": "UniProtKB:P08195"
}